{
  "gene_symbol": "SMYD4",
  "gene": "UniProtKB:Q8IYR2",
  "term_label": "cytoplasm",
  "term_id": "GO:0005737",
  "gene_name": "SET and MYND domain-containing protein 4"
}